long-chain-fatty-acyl-CoA reductase activity [GO:0050062] (molecular function) Sources: RHEA:15437 Note: Together with GO:0047474, forms a fatty acid reductase system which produces the substrate of GO:0047646, thus being part of the bacterial luciferase system. Relationships: is a type of GO:0016620 Also known as: long-chain fatty acyl CoA reductase activity, long-chain fatty acyl-CoA reductase activity, long-chain-fatty-acyl-CoA luciferin component reductase activity, acyl coenzyme A reductase activity Definition: Catalysis of the reaction: a long-chain fatty aldehyde + CoA + NADP+ = a long-chain fatty acyl-CoA + NADPH.